{
  "term_label": "Unknown molecular function",
  "gene": "UniProtKB:P0DTL6",
  "term_id": "UNKNOWN:0001",
  "gene_symbol": "ZFTRAF1",
  "gene_name": "Zinc finger TRAF-type-containing protein 1"
}